{
  "gene_name": "Fructose-bisphosphate aldolase B",
  "term_id": "GO:0004332",
  "gene_symbol": "ALDOB",
  "term_label": "fructose-bisphosphate aldolase activity",
  "gene": "UniProtKB:P05062"
}